positive regulation of female receptivity, post-mating [GO:0046009] (biological process) Sources: GOC:go_curators Also known as: up regulation of female receptivity, post-mating, up-regulation of female receptivity, post-mating, upregulation of female receptivity, post-mating, activation of female receptivity, post-mating, stimulation of female receptivity, post-mating Relationships: is a type of positive regulation of female receptivity [GO:0045925]; is_a regulation of female receptivity, post-mating [GO:0046008] Definition: Any process that increases the receptiveness of a female to male advances subsequent to mating.